leucocyanidin oxygenase activity [GO:0050589] (molecular function) Also known as: anthocyanidin synthase activity, leucoanthocyanidin dioxygenase activity, leucoanthocyanidin hydroxylase, leucocyanidin,2-oxoglutarate:oxygen oxidoreductase activity Sources: EC:1.14.20.4 Definition: Catalysis of the reaction: leucocyanidin + 2-oxoglutarate + O2 = cis- or trans-dihydroquercetin + succinate + CO2 + 2 H2O. Relationships: is a type of 2-oxoglutarate-dependent dioxygenase activity [GO:0016706]